{
  "gene_symbol": "SVIL",
  "gene": "UniProtKB:O95425",
  "gene_name": "Supervillin",
  "term_label": "actin filament severing",
  "term_id": "GO:0051014"
}